{
  "gene_name": "CaM kinase-like vesicle-associated protein",
  "term_label": "calcium/calmodulin-dependent protein kinase activity",
  "gene_symbol": "CAMKV",
  "gene": "UniProtKB:Q8NCB2",
  "term_id": "GO:0004683"
}